{
  "gene": "UniProtKB:P25963",
  "gene_name": "NF-kappa-B inhibitor alpha",
  "term_id": "GO:0051059",
  "term_label": "NF-kappaB binding",
  "gene_symbol": "NFKBIA"
}